{
  "gene_symbol": "FGFR2",
  "gene_name": "Fibroblast growth factor receptor 2",
  "term_id": "GO:0001525",
  "term_label": "angiogenesis",
  "gene": "UniProtKB:P21802"
}